ectexine [GO:0043669] (cellular component) References: PMID:28904424 Note: Note that ectexine is distinguished on staining properties; compare with 'sexine ; GO:0043673'. See also 'endexine ; GO:0043671'. Definition: The outer part of the exine, which stains positively with basic fuchsin in optical microscopy and has higher electron density in conventionally prepared TEM sections. Relationships: is a type of cellular anatomical structure [GO:0110165]; is part of exine [GO:0043668]